{
  "term_label": "cardiac muscle cell action potential involved in contraction",
  "gene_symbol": "SCN2B",
  "gene_name": "Sodium channel subunit beta-2",
  "term_id": "GO:0086002",
  "gene": "UniProtKB:O60939"
}